{
  "term_id": "GO:0005815",
  "gene_name": "G1_S-specific cyclin-E2",
  "gene": "UniProtKB:O96020",
  "gene_symbol": "CCNE2",
  "term_label": "microtubule organizing center"
}